methylammonium transmembrane transport [GO:0072489] (biological process) Relationships: is a type of GO:0015843; is a type of transmembrane transport [GO:0055085] Sources: GOC:mah Also known as: methylammonium membrane transport Definition: The process in which methylammonium is transported across a membrane. Note: Note that this term is not intended for use in annotating lateral movement within membranes.